phosphatidylinositol-3,5-bisphosphate 5-phosphatase activity [GO:0043813] (molecular function) Definition: Catalysis of the reaction: a 1,2-diacyl-sn-glycero-3-phospho-(1D-myo-inositol-3,5-bisphosphate) + H2O = a 1,2-diacyl-sn-glycero-3-phospho-(1D-myo-inositol-3-phosphate) + phosphate. References: PMID:10806194, PMID:16607019 Sources: RHEA:32955 Also known as: phosphatidylinositol 3,5-bisphosphate 5-phosphatase activity Relationships: is a type of phosphatidylinositol phosphate 5-phosphatase activity [GO:0034595]; is a type of phosphatidylinositol-3,5-bisphosphate phosphatase activity [GO:0106018]; BFO_0000050 phosphatidylinositol-3-phosphate biosynthetic process [GO:0036092]